{
  "gene_symbol": "CACNG7",
  "term_label": "voltage-gated calcium channel activity",
  "term_id": "GO:0005245",
  "gene_name": "Voltage-dependent calcium channel gamma-7 subunit",
  "gene": "UniProtKB:P62955"
}